{
  "gene_name": "Estrogen receptor",
  "gene_symbol": "ESR1",
  "term_label": "estrogen response element binding",
  "term_id": "GO:0034056",
  "gene": "UniProtKB:P03372"
}